{
  "gene_name": "Golgin subfamily A member 8J",
  "gene": "UniProtKB:A6NMD2",
  "term_id": "GO:0032580",
  "gene_symbol": "GOLGA8J",
  "term_label": "Golgi cisterna membrane"
}